2-pyrone-4,6-dicarboxylate lactonase activity [GO:0047554] (molecular function) Also known as: 2-pyrone-4,6-dicarboxylate lactonohydrolase activity Sources: EC:3.1.1.57, RHEA:10644 Definition: Catalysis of the reaction: 2-oxo-2H-pyran-4,6-dicarboxylate + H2O = 4-carboxy-2-hydroxyhexa-2,4-dienedioate + H+. Relationships: is a type of carboxylic ester hydrolase activity [GO:0052689]